{
  "term_id": "UNKNOWN:0001",
  "gene": "UniProtKB:O60880",
  "gene_symbol": "SH2D1A",
  "term_label": "Unknown molecular function",
  "gene_name": "SH2 domain-containing protein 1A"
}